regulation of cytoplasmic translational elongation [GO:1900247] (biological process) Sources: GOC:TermGenie Subtypes: GO:0140018, negative regulation of cytoplasmic translational elongation [GO:1900248], GO:1900249, regulation of cytoplasmic translational elongation through polyproline stretches [GO:1903270] Relationships: is a type of GO:0006448; regulates cytoplasmic translational elongation [GO:0002182] Definition: Any process that modulates the frequency, rate or extent of cytoplasmic translational elongation.